{
  "gene_symbol": "TBCEL",
  "gene": "UniProtKB:Q5QJ74",
  "gene_name": "Tubulin-specific chaperone cofactor E-like protein",
  "term_label": "cytoplasm",
  "term_id": "GO:0005737"
}